{
  "gene_name": "Ras-related C3 botulinum toxin substrate 2",
  "term_id": "GO:0007015",
  "term_label": "actin filament organization",
  "gene_symbol": "RAC2",
  "gene": "UniProtKB:P15153"
}